{
  "gene_name": "H(+)_Cl(-) exchange transporter 3",
  "gene": "UniProtKB:P51790",
  "term_label": "Golgi apparatus",
  "gene_symbol": "CLCN3",
  "term_id": "GO:0005794"
}